{
  "gene_name": "Ryanodine receptor 2",
  "gene": "UniProtKB:Q92736",
  "term_id": "GO:0006941",
  "gene_symbol": "RYR2",
  "term_label": "striated muscle contraction"
}